integrin alpha8-beta1 complex [GO:0034678] (cellular component) References: PMID:12297042 Relationships: is a type of integrin complex [GO:0008305] Definition: An integrin complex that comprises one alpha8 subunit and one beta1 subunit. Also known as: alpha8-beta1 integrin complex, ITGA8-ITGB1 complex